{
  "term_id": "UNKNOWN:0002",
  "gene_symbol": "TBKBP1",
  "gene": "UniProtKB:A7MCY6",
  "gene_name": "TANK-binding kinase 1-binding protein 1",
  "term_label": "Unknown biological process"
}